{
  "gene": "UniProtKB:Q9Y5F2",
  "gene_name": "Protocadherin beta-11",
  "gene_symbol": "PCDHB11",
  "term_label": "cell adhesion",
  "term_id": "GO:0007155"
}